{
  "gene": "UniProtKB:Q12860",
  "term_label": "axon guidance",
  "gene_symbol": "CNTN1",
  "term_id": "GO:0007411",
  "gene_name": "Contactin-1"
}